{
  "gene": "UniProtKB:P51693",
  "gene_symbol": "APLP1",
  "gene_name": "Amyloid beta precursor like protein 1",
  "term_label": "alpha-2C adrenergic receptor binding",
  "term_id": "GO:0031696"
}